{
  "term_id": "GO:0030687",
  "gene": "UniProtKB:Q9UKD2",
  "term_label": "preribosome, large subunit precursor",
  "gene_name": "mRNA turnover protein 4 homolog",
  "gene_symbol": "MRTO4"
}